{
  "gene_name": "Fatty acid-binding protein, adipocyte",
  "gene_symbol": "FABP4",
  "term_label": "cytosol",
  "gene": "UniProtKB:P15090",
  "term_id": "GO:0005829"
}